{
  "gene_name": "Myosin-14",
  "gene": "UniProtKB:Q7Z406",
  "gene_symbol": "MYH14",
  "term_id": "UNKNOWN:0001",
  "term_label": "Unknown molecular function"
}